cell wall macromolecule catabolic process involved in cytogamy [GO:0032219] (biological process) Also known as: cell wall macromolecule catabolic process during cytogamy Relationships: is a type of cell wall macromolecule catabolic process [GO:0016998]; is part of GO:0000755 Definition: The chemical reactions and pathways resulting in the breakdown of macromolecules forming part of a cell wall that contribute to cytogamy. Sources: GOC:mah